{
  "gene_symbol": "HOXB13",
  "gene": "UniProtKB:Q92826",
  "term_label": "Unknown cellular component",
  "gene_name": "Homeobox protein Hox-B13",
  "term_id": "UNKNOWN:0003"
}